{
  "gene": "UniProtKB:O43613",
  "gene_symbol": "HCRTR1",
  "term_label": "cellular response to hormone stimulus",
  "term_id": "GO:0032870",
  "gene_name": "Orexin_Hypocretin receptor type 1"
}